{
  "gene_symbol": "HEMGN",
  "term_label": "nucleoplasm",
  "term_id": "GO:0005654",
  "gene": "UniProtKB:Q9BXL5",
  "gene_name": "Hemogen"
}